{
  "gene_symbol": "CIAO3",
  "term_id": "UNKNOWN:0002",
  "gene_name": "Cytosolic iron-sulfur assembly component 3",
  "gene": "UniProtKB:Q9H6Q4",
  "term_label": "Unknown biological process"
}